{
  "gene": "UniProtKB:Q494X3",
  "gene_name": "Zinc finger protein 404",
  "gene_symbol": "ZNF404",
  "term_label": "RNA polymerase II transcription regulatory region sequence-specific DNA binding",
  "term_id": "GO:0000977"
}